positive regulation of convergent extension involved in neural plate elongation [GO:1904132] (BP) Definition: Any process that activates or increases the frequency, rate or extent of convergent extension involved in neural plate elongation. References: PMID:24892953 Sources: GOC:TermGenie, GOC:dph, GO_REF:0000058 Also known as: up regulation of convergent extension involved in neural plate elongation, up-regulation of convergent extension involved in neural plate elongation, upregulation of convergent extension involved in neural plate elongation, activation of convergent extension involved in neural plate elongation Relationships: is a type of positive regulation of convergent extension involved in gastrulation [GO:1904105]; is a type of regulation of convergent extension involved in neural plate elongation [GO:1904130]; positively regulates GO:0022007